{
  "gene_symbol": "ARHGEF18",
  "gene_name": "Rho guanine nucleotide exchange factor 18",
  "gene": "UniProtKB:Q6ZSZ5",
  "term_id": "GO:0007264",
  "term_label": "small GTPase-mediated signal transduction"
}